{
  "term_id": "UNKNOWN:0001",
  "gene": "UniProtKB:Q9Y3B9",
  "gene_symbol": "RRP15",
  "term_label": "Unknown molecular function",
  "gene_name": "RRP15-like protein"
}